cellular defense response [GO:0006968] (biological process) Sources: GOC:ebc Definition: A defense response that is mediated by cells. Relationships: is a type of defense response [GO:0006952] Regulation: RO_0002211 by GO:0010185; positively regulated by positive regulation of cellular defense response [GO:0010186]; negatively regulated by GO:0051245 Also known as: cellular defence response, intracellular defence response, intracellular defense response